{
  "gene": "UniProtKB:Q3MIT2",
  "term_id": "GO:0009982",
  "term_label": "pseudouridine synthase activity",
  "gene_name": "tRNA pseudouridine synthase Pus10",
  "gene_symbol": "PUS10"
}